{
  "gene_symbol": "FMO2",
  "gene_name": "Flavin-containing monooxygenase 2",
  "gene": "UniProtKB:Q99518",
  "term_label": "Unknown cellular component",
  "term_id": "UNKNOWN:0003"
}